{
  "gene_name": "Metallothionein-1A",
  "term_label": "cellular response to copper ion",
  "gene_symbol": "MT1A",
  "term_id": "GO:0071280",
  "gene": "UniProtKB:P04731"
}